{
  "term_id": "GO:0000981",
  "gene_name": "Paired box protein Pax-3",
  "gene_symbol": "PAX3",
  "term_label": "DNA-binding transcription factor activity, RNA polymerase II-specific",
  "gene": "UniProtKB:P23760"
}